cellular response to antibiotic [GO:0071236] (biological process) Sources: GOC:mah Relationships: is a type of response to antibiotic [GO:0046677]; is a type of cellular response to chemical stimulus [GO:0070887] Subtypes: GO:0035984, cellular response to bacteriocin [GO:0071237], GO:0071238, cellular response to streptomycin [GO:0071239], cellular response to actinomycin D [GO:0072717] Definition: Any process that results in a change in state or activity of a cell (in terms of movement, secretion, enzyme production, gene expression, etc.) as a result of an antibiotic stimulus. An antibiotic is a chemical substance produced by a microorganism which has the capacity to inhibit the growth of or to kill other microorganisms.